{
  "gene_name": "Putative coiled-coil domain-containing protein 144 N-terminal-like",
  "term_label": "Unknown molecular function",
  "gene": "UniProtKB:Q6NUI1",
  "gene_symbol": "CCDC144NL",
  "term_id": "UNKNOWN:0001"
}